{
  "gene_symbol": "PTCH1",
  "term_label": "smoothened binding",
  "gene": "UniProtKB:Q13635",
  "term_id": "GO:0005119",
  "gene_name": "Protein patched homolog 1"
}